{
  "gene_symbol": "PSMA6",
  "gene": "UniProtKB:P60900",
  "term_id": "GO:0019773",
  "term_label": "proteasome core complex, alpha-subunit complex",
  "gene_name": "Proteasome subunit alpha type-6"
}